diamine N-acetyltransferase complex [GO:1990235] (cellular component) References: PMID:8077207 Sources: GOC:bhm Also known as: SAT complex, SAT tetramer, spermidine acetyltransferase complex Definition: A protein complex which is capable of diamine N-acetyltransferase activity. Relationships: is a type of acetyltransferase complex [GO:1902493]; is part of cytosol [GO:0005829]